{
  "term_label": "thiamine pyrophosphate binding",
  "term_id": "GO:0030976",
  "gene": "UniProtKB:Q9UJ83",
  "gene_name": "2-hydroxyacyl-CoA lyase 1",
  "gene_symbol": "HACL1"
}